{
  "gene": "UniProtKB:Q17RY6",
  "term_id": "UNKNOWN:0001",
  "gene_symbol": "LY6K",
  "gene_name": "Lymphocyte antigen 6K",
  "term_label": "Unknown molecular function"
}